{
  "term_label": "peptide cross-linking",
  "gene": "UniProtKB:P21980",
  "term_id": "GO:0018149",
  "gene_name": "Protein-glutamine gamma-glutamyltransferase 2",
  "gene_symbol": "TGM2"
}